macrophage fusion [GO:0034238] (biological process) Definition: The binding and fusion of a macrophage to one or more other cells to form a multinucleated cell. Sources: GOC:sl Relationships: is a type of syncytium formation by plasma membrane fusion [GO:0000768] Regulation: regulated by regulation of macrophage fusion [GO:0034239]; negatively regulated by negative regulation of macrophage fusion [GO:0034240]; positively regulated by positive regulation of macrophage fusion [GO:0034241]